{
  "gene_name": "Integrin beta-1",
  "gene": "UniProtKB:P05556",
  "term_id": "GO:0019901",
  "gene_symbol": "ITGB1",
  "term_label": "protein kinase binding"
}